{
  "term_id": "GO:0000785",
  "gene_name": "Estrogen receptor",
  "gene_symbol": "ESR1",
  "gene": "UniProtKB:P03372",
  "term_label": "chromatin"
}